{
  "gene_name": "Cyclic nucleotide-gated cation channel beta-1",
  "gene_symbol": "CNGB1",
  "term_id": "GO:0001895",
  "term_label": "retina homeostasis",
  "gene": "UniProtKB:Q14028"
}